{
  "gene": "UniProtKB:Q9P219",
  "term_label": "centrosome",
  "gene_symbol": "CCDC88C",
  "term_id": "GO:0005813",
  "gene_name": "Protein Daple"
}